{
  "gene_name": "Torsin-2A",
  "term_id": "GO:0005788",
  "gene": "UniProtKB:Q5JU69",
  "term_label": "endoplasmic reticulum lumen",
  "gene_symbol": "TOR2A"
}